{
  "gene": "UniProtKB:Q496Y0",
  "term_label": "Unknown biological process",
  "term_id": "UNKNOWN:0002",
  "gene_name": "LON peptidase N-terminal domain and RING finger protein 3",
  "gene_symbol": "LONRF3"
}